{
  "term_label": "RNA polymerase II transcription regulatory region sequence-specific DNA binding",
  "term_id": "GO:0000977",
  "gene_symbol": "PEG3",
  "gene_name": "Paternally-expressed gene 3 protein",
  "gene": "UniProtKB:Q9GZU2"
}